{
  "gene": "UniProtKB:Q8N1D5",
  "term_id": "UNKNOWN:0002",
  "term_label": "Unknown biological process",
  "gene_symbol": "CFAP107",
  "gene_name": "Cilia- and flagella-associated protein 107"
}